{
  "term_id": "GO:0006357",
  "term_label": "regulation of transcription by RNA polymerase II",
  "gene_name": "Zinc finger protein 585A",
  "gene": "UniProtKB:Q6P3V2",
  "gene_symbol": "ZNF585A"
}